{
  "term_id": "GO:0000786",
  "gene_symbol": "H2BW2",
  "gene": "UniProtKB:P0C1H6",
  "gene_name": "Histone H2B type F-M",
  "term_label": "nucleosome"
}